{
  "gene_symbol": "FAM106A",
  "gene": "UniProtKB:Q4KMX7",
  "gene_name": "Protein FAM106A",
  "term_id": "UNKNOWN:0002",
  "term_label": "Unknown biological process"
}